positive regulation of corticosterone secretion [GO:2000854] (BP) Sources: GOC:sl Relationships: is a type of positive regulation of glucocorticoid secretion [GO:2000851]; is a type of regulation of corticosterone secretion [GO:2000852]; positively regulates corticosterone secretion [GO:0035934] Definition: Any process that activates or increases the frequency, rate or extent of corticosterone secretion.